natriuretic peptide receptor activity [GO:0016941] (molecular function) Sources: GOC:mah, GOC:signaling Relationships: is a type of peptide receptor activity [GO:0001653] Definition: Combining with a natriuretic peptide and transmitting the signal to initiate a change in cell activity.